cutin transport [GO:0080051] (biological process) Definition: The directed movement of cutin into, out of or within a cell, or between cells, by means of some agent such as a transporter or pore. Cutin, which consists of C16-18 fatty acids, is the major component of the cuticle that covers the plant surface. References: PMID:17951461 Relationships: is a type of transport [GO:0006810]